alkyl hydroperoxide reductase activity [GO:0008785] (molecular function) Relationships: is a type of oxidoreductase activity, acting on a sulfur group of donors, NAD(P) as acceptor [GO:0016668] Definition: Catalysis of the reaction: octane hydroperoxide + NADH + H+ = H2O + NAD+ + 1-octanol. Sources: GOC:curators